{
  "term_label": "bicellular tight junction",
  "gene_symbol": "CGN",
  "gene_name": "Cingulin",
  "term_id": "GO:0005923",
  "gene": "UniProtKB:Q9P2M7"
}